{
  "term_label": "RNA binding",
  "gene_symbol": "RALYL",
  "gene_name": "RNA-binding Raly-like protein",
  "gene": "UniProtKB:Q86SE5",
  "term_id": "GO:0003723"
}